riboflavin synthase complex [GO:0009349] (CC) References: PMID:18298940 Definition: An flavoprotein that catalyzes the reaction the breakdown of dimethyl(ribityl)lumazine to form riboflavin and ribitylamino-amino-dihydroxypyrimidine. Relationships: is a type of transferase complex [GO:1990234]